type 2 cysteinyl leukotriene receptor binding [GO:0031747] (molecular function) Definition: Binding to a type 2 cysteinyl leukotriene receptor. Relationships: is a type of cysteinyl leukotriene receptor binding [GO:0031745] Sources: GOC:mah, GOC:nln Also known as: type 2 cysteinyl leukotriene receptor ligand